UCU codon-amino acid adaptor activity [GO:0033405] (molecular function) Also known as: TCT codon-amino acid adaptor activity, serine tRNA Definition: A triplet codon-amino acid adaptor activity that recognizes a UCU codon. Note: Note that in the standard genetic code, TCT codes for serine. Relationships: is a type of triplet codon-amino acid adaptor activity [GO:0030533] Sources: GOC:mah